{
  "gene": "UniProtKB:P0DQW0",
  "term_label": "nucleus",
  "gene_symbol": "ZC3H11C",
  "gene_name": "Zinc finger CCCH domain-containing protein 11C",
  "term_id": "GO:0005634"
}